{
  "term_id": "GO:0005783",
  "term_label": "endoplasmic reticulum",
  "gene_symbol": "LTC4S",
  "gene_name": "Leukotriene C4 synthase",
  "gene": "UniProtKB:Q16873"
}